{
  "gene_symbol": "C5orf60",
  "term_id": "UNKNOWN:0003",
  "gene": "UniProtKB:A6NFR6",
  "term_label": "Unknown cellular component",
  "gene_name": "Uncharacterized protein C5orf60"
}